threonine racemase activity [GO:0018114] (molecular function) Relationships: is a type of GO:0047661 Sources: EC:5.1.1.6, RHEA:13913 Definition: Catalysis of the reaction: L-threonine = D-threonine.